{
  "gene": "UniProtKB:Q5FWF4",
  "term_id": "GO:0031297",
  "term_label": "replication fork processing",
  "gene_symbol": "ZRANB3",
  "gene_name": "DNA annealing helicase and endonuclease ZRANB3"
}